{
  "term_label": "extracellular space",
  "gene_symbol": "MICB",
  "gene_name": "MHC class I polypeptide-related sequence B",
  "term_id": "GO:0005615",
  "gene": "UniProtKB:Q29980"
}